programmed necrotic cell death in response to starvation [GO:0097385] (biological process) References: PMID:13679856 Sources: GOC:mtg_apoptosis, GOC:pg Definition: A programmed necrotic cell death occurring as a result of a starvation stimulus (deprivation of nourishment). Also known as: necrotic cell death in response to starvation Relationships: is a type of response to starvation [GO:0042594]; is a type of programmed necrotic cell death [GO:0097300]